{
  "gene": "UniProtKB:Q9BQS8",
  "gene_name": "FYVE and coiled-coil domain-containing protein 1",
  "term_id": "GO:0005770",
  "term_label": "late endosome",
  "gene_symbol": "FYCO1"
}